{
  "gene_symbol": "FAM234B",
  "term_label": "Unknown cellular component",
  "term_id": "UNKNOWN:0003",
  "gene": "UniProtKB:A2RU67",
  "gene_name": "Protein FAM234B"
}